{
  "gene_name": "Homeobox protein Nkx-2.2",
  "term_label": "DNA-binding transcription factor activity, RNA polymerase II-specific",
  "term_id": "GO:0000981",
  "gene": "UniProtKB:O95096",
  "gene_symbol": "NKX2-2"
}